{
  "gene_symbol": "STAT3",
  "term_id": "GO:0090575",
  "term_label": "RNA polymerase II transcription regulator complex",
  "gene": "UniProtKB:P40763",
  "gene_name": "Signal transducer and activator of transcription 3"
}